aldehyde ferredoxin oxidoreductase activity [GO:0033726] (MF) Definition: Catalysis of the reaction: an aldehyde + H2O + 2 oxidized ferredoxin = an acid + 2 H+ + 2 reduced ferredoxin. Sources: EC:1.2.7.5 Also known as: AOR, aldehyde:ferredoxin oxidoreductase activity, tungsten-containing aldehyde ferredoxin oxidoreductase activity Relationships: is a type of GO:0016625